{
  "gene_name": "Shiftless antiviral inhibitor of ribosomal frameshifting protein",
  "gene": "UniProtKB:Q9NUL5",
  "term_label": "viral translational frameshifting",
  "term_id": "GO:0075523",
  "gene_symbol": "SHFL"
}